{
  "gene": "UniProtKB:P13640",
  "term_label": "nucleus",
  "gene_symbol": "MT1G",
  "term_id": "GO:0005634",
  "gene_name": "Metallothionein-1G"
}